{
  "gene": "UniProtKB:Q9C0C6",
  "term_id": "UNKNOWN:0001",
  "term_label": "Unknown molecular function",
  "gene_name": "CLOCK-interacting pacemaker",
  "gene_symbol": "CIPC"
}